{
  "term_label": "ubiquitin activating enzyme activity",
  "gene_name": "Ubiquitin-like modifier-activating enzyme 6",
  "gene_symbol": "UBA6",
  "gene": "UniProtKB:A0AVT1",
  "term_id": "GO:0004839"
}